{
  "term_label": "GTP binding",
  "gene_name": "ADP-ribosylation factor-like protein 5A",
  "term_id": "GO:0005525",
  "gene_symbol": "ARL5A",
  "gene": "UniProtKB:Q9Y689"
}